{
  "term_id": "GO:0034599",
  "gene_name": "Glutathione peroxidase 6",
  "gene_symbol": "GPX6",
  "term_label": "cellular response to oxidative stress",
  "gene": "UniProtKB:P59796"
}